positive regulation of store-operated calcium channel activity [GO:1901341] (biological process) Subtypes: GO:0032237 Definition: Any process that activates or increases the frequency, rate or extent of store-operated calcium channel activity. Relationships: is a type of regulation of store-operated calcium channel activity [GO:1901339]; is a type of positive regulation of cation channel activity [GO:2001259]; positively regulates store-operated calcium channel activity [GO:0015279] Sources: GOC:TermGenie Also known as: up regulation of store-operated calcium channel activity, up-regulation of store-operated calcium channel activity, upregulation of store-operated calcium channel activity, activation of store-operated calcium channel activity